{
  "term_id": "UNKNOWN:0003",
  "gene_symbol": "EEF1A1P5",
  "term_label": "Unknown cellular component",
  "gene": "UniProtKB:Q5VTE0",
  "gene_name": "Putative elongation factor 1-alpha-like 3"
}